{
  "gene_symbol": "EML3",
  "gene": "UniProtKB:Q32P44",
  "term_label": "microtubule binding",
  "gene_name": "Echinoderm microtubule-associated protein-like 3",
  "term_id": "GO:0008017"
}